tooth eruption [GO:0044691] (biological process) Definition: The tooth development process in which the teeth enter the mouth and become visible. Sources: Wikipedia:Tooth_eruption Relationships: is a type of anatomical structure development [GO:0048856]; is part of odontogenesis [GO:0042476]